cobalamin metabolic process [GO:0009235] (biological process) Also known as: cobalamin metabolism, vitamin B12 metabolic process, vitamin B12 metabolism, vitamin B12 reduction Definition: The chemical reactions and pathways involving cobalamin (vitamin B12), a water-soluble vitamin characterized by possession of a corrin nucleus containing a cobalt atom. Relationships: is a type of tetrapyrrole metabolic process [GO:0033013] Sources: GOC:go_curators Regulation: regulated by regulation of cobalamin metabolic process [GO:0106064]; positively regulated by positive regulation of cobalamin metabolic process [GO:0106121]; negatively regulated by GO:0106122 Subtypes: GO:0009236, cobalamin catabolic process [GO:0042366]